{
  "term_id": "GO:0005549",
  "gene_name": "Olfactory receptor 5B3",
  "gene": "UniProtKB:Q8NH48",
  "term_label": "odorant binding",
  "gene_symbol": "OR5B3"
}